{
  "gene": "UniProtKB:Q8NAA5",
  "gene_name": "Leucine-rich repeat-containing protein 75A",
  "term_id": "GO:0043161",
  "gene_symbol": "LRRC75A",
  "term_label": "proteasome-mediated ubiquitin-dependent protein catabolic process"
}